induced systemic resistance, jasmonic acid mediated signaling pathway [GO:0009864] (biological process) Relationships: is a type of GO:0002218; is a type of immune effector process [GO:0002252]; is a type of GO:0009867; is part of induced systemic resistance [GO:0009682] Definition: The series of molecular signals mediated by jasmonic acid involved in induced systemic resistance. Also known as: induced systemic resistance, jasmonic acid mediated signalling pathway, jasmonic acid mediated signaling pathway (induced systemic resistance) Sources: GOC:jy